{
  "gene_name": "Phosphoinositide 3-kinase regulatory subunit 4",
  "term_id": "GO:0006623",
  "gene_symbol": "PIK3R4",
  "gene": "UniProtKB:Q99570",
  "term_label": "protein targeting to vacuole"
}